{
  "gene": "UniProtKB:Q05BU3",
  "gene_name": "Putative protein FAM86JP",
  "term_id": "UNKNOWN:0002",
  "gene_symbol": "FAM86JP",
  "term_label": "Unknown biological process"
}